{
  "term_id": "GO:0003924",
  "gene_name": "Ribosome-releasing factor 2, mitochondrial",
  "gene": "UniProtKB:Q969S9",
  "gene_symbol": "GFM2",
  "term_label": "GTPase activity"
}